{
  "gene_name": "Sharpin",
  "gene": "UniProtKB:Q9H0F6",
  "gene_symbol": "SHARPIN",
  "term_id": "GO:0043130",
  "term_label": "ubiquitin binding"
}